{
  "gene": "UniProtKB:P26715",
  "term_label": "negative regulation of natural killer cell mediated cytotoxicity",
  "gene_symbol": "KLRC1",
  "term_id": "GO:0045953",
  "gene_name": "NKG2-A_NKG2-B type II integral membrane protein"
}